hindbrain tangential cell migration [GO:0021934] (biological process) Sources: GOC:cls, GOC:dgh, GOC:dph, GOC:jid, GO_REF:0000021 Subtypes: GO:0021935, brainstem precerebellar neuron precursor migration [GO:0021949] Relationships: is a type of cell migration in hindbrain [GO:0021535] Definition: The migration of a cell in the hindbrain in which cells move orthogonal to the direction of radial migration. Also known as: hindbrain neurophilic migration